T cell activation involved in immune response [GO:0002286] (BP) Subtypes: alpha-beta T cell activation involved in immune response [GO:0002287], gamma-delta T cell activation involved in immune response [GO:0002290], T cell activation via T cell receptor contact with antigen bound to MHC molecule on antigen presenting cell [GO:0002291], T cell differentiation involved in immune response [GO:0002292], T cell proliferation involved in immune response [GO:0002309] Sources: GOC:add, ISBN:0781735149 Relationships: is a type of lymphocyte activation involved in immune response [GO:0002285]; is_a T cell activation [GO:0042110] Definition: The change in morphology and behavior of a mature or immature T cell resulting from exposure to a mitogen, cytokine, chemokine, cellular ligand, or an antigen for which it is specific, leading to the initiation or perpetuation of an immune response. Also known as: T cell activation during immune response, T lymphocyte activation during immune response, T-cell activation during immune response, T-lymphocyte activation during immune response